chloroplast mRNA processing [GO:0010239] (biological process) Definition: Steps involved in processing precursor RNAs arising from transcription of operons in the chloroplast genome into mature mRNAs. References: PMID:9648738 Sources: GOC:tb Relationships: is a type of mRNA processing [GO:0006397]; is a type of chloroplast RNA processing [GO:0031425]; occurs in chloroplast [GO:0009507]